{
  "term_id": "GO:0005634",
  "gene_name": "Chromodomain-helicase-DNA-binding protein 4",
  "gene": "UniProtKB:Q14839",
  "term_label": "nucleus",
  "gene_symbol": "CHD4"
}